{
  "gene_name": "NCK-interacting protein with SH3 domain",
  "gene": "UniProtKB:Q9NZQ3",
  "term_id": "GO:0006897",
  "gene_symbol": "NCKIPSD",
  "term_label": "endocytosis"
}